{
  "gene_symbol": "FGF4",
  "term_id": "GO:0022008",
  "gene": "UniProtKB:P08620",
  "gene_name": "Fibroblast growth factor 4",
  "term_label": "neurogenesis"
}